{
  "gene_symbol": "STK25",
  "gene": "UniProtKB:O00506",
  "gene_name": "Serine_threonine-protein kinase 25",
  "term_id": "GO:0004674",
  "term_label": "protein serine/threonine kinase activity"
}